{
  "gene_name": "Uncharacterized protein C1orf131",
  "term_id": "UNKNOWN:0002",
  "gene_symbol": "C1orf131",
  "term_label": "Unknown biological process",
  "gene": "UniProtKB:Q8NDD1"
}